{
  "term_id": "GO:0016581",
  "term_label": "NuRD complex",
  "gene": "UniProtKB:Q92769",
  "gene_symbol": "HDAC2",
  "gene_name": "Histone deacetylase 2"
}